positive regulation of male mating behavior [GO:1902437] (biological process) Subtypes: positive regulation of turning behavior involved in mating [GO:0061095] Also known as: up regulation of male mating behavior, up-regulation of male mating behavior, upregulation of male mating behavior, activation of male mating behavior References: PMID:24089208 Sources: GOC:TermGenie Definition: Any process that activates or increases the frequency, rate or extent of male mating behavior. Relationships: is a type of positive regulation of behavior [GO:0048520]; is a type of regulation of male mating behavior [GO:1902435]; is a type of GO:2000243; RO_0002213 GO:0060179